{
  "term_label": "Unknown molecular function",
  "term_id": "UNKNOWN:0001",
  "gene": "UniProtKB:Q8N3X6",
  "gene_symbol": "LCORL",
  "gene_name": "Ligand-dependent nuclear receptor corepressor-like protein"
}